{
  "gene_name": "U4_U6 small nuclear ribonucleoprotein Prp3",
  "gene_symbol": "PRPF3",
  "gene": "UniProtKB:O43395",
  "term_id": "GO:0000398",
  "term_label": "mRNA splicing, via spliceosome"
}